positive regulation of phagosome maturation [GO:1905164] (biological process) Sources: GOC:PARL, GOC:TermGenie, GOC:bf, GO_REF:0000058 Also known as: up regulation of phagosome maturation, up-regulation of phagosome maturation, upregulation of phagosome maturation, activation of phagosome maturation Relationships: is a type of positive regulation of organelle organization [GO:0010638]; is a type of regulation of phagosome maturation [GO:1905162]; positively regulates phagosome maturation [GO:0090382] Definition: Any process that activates or increases the frequency, rate or extent of phagosome maturation.